{
  "gene": "UniProtKB:Q50LG9",
  "gene_symbol": "LRRC24",
  "gene_name": "Leucine-rich repeat-containing protein 24",
  "term_id": "GO:0009897",
  "term_label": "external side of plasma membrane"
}